{
  "term_label": "microtubule cytoskeleton",
  "gene_symbol": "SEPTIN11",
  "gene": "UniProtKB:Q9NVA2",
  "gene_name": "Septin-11",
  "term_id": "GO:0015630"
}